lysosomal proton-transporting V-type ATPase complex [GO:0046611] (cellular component) Definition: A proton-transporting two-sector ATPase complex found in the lysosomal membrane, where it acts as a proton pump to mediate acidification of the lysosomal lumen. References: PMID:16449553 Sources: GOC:mah, ISBN:0716743663 Also known as: lysosomal membrane hydrogen-transporting ATPase, lysosomal hydrogen-translocating V-type ATPase complex Relationships: is a type of vacuolar proton-transporting V-type ATPase complex [GO:0016471]; is part of GO:0005765